regulation of alkane biosynthetic process [GO:1901577] (biological process) Definition: Any process that modulates the frequency, rate or extent of alkane biosynthetic process. Sources: GOC:TermGenie Also known as: regulation of alkane anabolism, regulation of alkane biosynthesis, regulation of alkane formation, regulation of alkane synthesis Relationships: is a type of regulation of biosynthetic process [GO:0009889]; regulates alkane biosynthetic process [GO:0043447] Subtypes: regulation of methane biosynthetic process from dimethylamine [GO:1900318], GO:1900330, regulation of methane biosynthetic process from 3-(methylthio)propionic acid [GO:1900333], regulation of methane biosynthetic process from carbon monoxide [GO:1900336], GO:1900339, regulation of methane biosynthetic process from dimethyl sulfide [GO:1900342], regulation of methane biosynthetic process from methanethiol [GO:1900345], regulation of methane biosynthetic process from methylamine [GO:1900348], regulation of tridecane biosynthetic process [GO:1900884], regulation of pentadecane biosynthetic process [GO:1900887], GO:1900896, negative regulation of alkane biosynthetic process [GO:1901578], GO:1901579